{
  "term_id": "GO:0004984",
  "gene_symbol": "OR5B3",
  "gene_name": "Olfactory receptor 5B3",
  "term_label": "olfactory receptor activity",
  "gene": "UniProtKB:Q8NH48"
}